{
  "gene_name": "Ankyrin repeat and LEM domain-containing protein 1",
  "gene_symbol": "ANKLE1",
  "term_id": "GO:0000712",
  "gene": "UniProtKB:Q8NAG6",
  "term_label": "resolution of meiotic recombination intermediates"
}